{
  "term_id": "GO:0006606",
  "gene": "UniProtKB:P61970",
  "term_label": "protein import into nucleus",
  "gene_name": "Nuclear transport factor 2",
  "gene_symbol": "NUTF2"
}